{
  "gene_symbol": "NCOA5",
  "gene_name": "Nuclear receptor coactivator 5",
  "term_id": "UNKNOWN:0001",
  "term_label": "Unknown molecular function",
  "gene": "UniProtKB:Q9HCD5"
}